{
  "gene": "UniProtKB:Q8WXK4",
  "gene_symbol": "ASB12",
  "term_id": "UNKNOWN:0002",
  "term_label": "Unknown biological process",
  "gene_name": "Ankyrin repeat and SOCS box protein 12"
}